{
  "term_label": "immune response",
  "gene_name": "Immunoglobulin lambda variable 2-18",
  "gene": "UniProtKB:A0A075B6J9",
  "gene_symbol": "IGLV2-18",
  "term_id": "GO:0006955"
}